detection of light stimulus involved in visual perception [GO:0050908] (biological process) Definition: The series of events involved in visual perception in which a light stimulus is received and converted into a molecular signal. Sources: GOC:ai, GOC:dos Relationships: is_a detection of light stimulus involved in sensory perception [GO:0050962]; BFO_0000050 visual perception [GO:0007601] Also known as: sensory detection of light during visual perception, sensory detection of light stimulus during visual perception, sensory transduction of light during visual perception, sensory transduction of light stimulus during visual perception, visual perception, detection of light stimulus, visual perception, sensory transduction during perception of light, visual perception, sensory transduction of light stimulus